{
  "gene_name": "Vacuolar protein sorting-associated protein 26B",
  "gene": "UniProtKB:Q4G0F5",
  "term_id": "GO:0006886",
  "term_label": "intracellular protein transport",
  "gene_symbol": "VPS26B"
}